{
  "gene_symbol": "GCDH",
  "gene_name": "Glutaryl-CoA dehydrogenase, mitochondrial",
  "term_label": "fatty acid beta-oxidation using acyl-CoA dehydrogenase",
  "gene": "UniProtKB:Q92947",
  "term_id": "GO:0033539"
}